{
  "term_label": "plasma membrane",
  "gene_name": "Epithelial membrane protein 2",
  "gene_symbol": "EMP2",
  "term_id": "GO:0005886",
  "gene": "UniProtKB:P54851"
}